{
  "term_label": "protein N-linked glycosylation",
  "gene_symbol": "DAD1",
  "term_id": "GO:0006487",
  "gene": "UniProtKB:P61803",
  "gene_name": "Dolichyl-diphosphooligosaccharide--protein glycosyltransferase subunit DAD1"
}